{
  "gene_symbol": "HAPLN4",
  "term_id": "GO:0045202",
  "term_label": "synapse",
  "gene": "UniProtKB:Q86UW8",
  "gene_name": "Hyaluronan and proteoglycan link protein 4"
}